{
  "term_id": "UNKNOWN:0002",
  "gene_name": "Zinc finger protein 862",
  "gene": "UniProtKB:O60290",
  "term_label": "Unknown biological process",
  "gene_symbol": "ZNF862"
}